{
  "gene_name": "Probable non-functional T cell receptor beta variable 17",
  "term_label": "plasma membrane",
  "gene": "UniProtKB:A0A087X0K7",
  "term_id": "GO:0005886",
  "gene_symbol": "TRBV17"
}